{
  "gene_symbol": "GJB4",
  "term_label": "cell-cell signaling",
  "term_id": "GO:0007267",
  "gene_name": "Gap junction beta-4 protein",
  "gene": "UniProtKB:Q9NTQ9"
}